{
  "gene_symbol": "PLEKHA4",
  "gene": "UniProtKB:Q9H4M7",
  "term_id": "GO:0090263",
  "gene_name": "Pleckstrin homology domain-containing family A member 4",
  "term_label": "positive regulation of canonical Wnt signaling pathway"
}